{
  "gene_name": "Fibroblast growth factor 12",
  "term_id": "GO:0017080",
  "term_label": "sodium channel regulator activity",
  "gene_symbol": "FGF12",
  "gene": "UniProtKB:P61328"
}